adenosine to inosine editing [GO:0006382] (biological process) Subtypes: tRNA wobble adenosine to inosine editing [GO:0002100] Definition: The conversion of an adenosine residue to inosine in an RNA molecule by deamination. Relationships: is a type of GO:0016553 References: PMID:11092837